negative regulation of compound eye photoreceptor cell differentiation [GO:0110118] (biological process) Definition: Any process that stops, prevents, or reduces the frequency, rate or extent of compound eye photoreceptor cell differentiation. Relationships: is a type of negative regulation of photoreceptor cell differentiation [GO:0046533]; is a type of regulation of compound eye photoreceptor cell differentiation [GO:0110116]; negatively regulates compound eye photoreceptor cell differentiation [GO:0001751] References: PMID:16377567 Sources: GOC:ha Subtypes: GO:0045677, negative regulation of R8 cell differentiation [GO:0045680]